outer membrane-bounded periplasmic space [GO:0030288] (cellular component) Relationships: is a type of periplasmic space [GO:0042597]; is part of cell envelope [GO:0030313] Also known as: outer membrane bounded periplasmic space, outer membrane-enclosed periplasmic space Sources: GOC:mlg, GOC:mtg_sensu Definition: The region between the inner (cytoplasmic or plasma) membrane and outer membrane of organisms with two membranes such as Gram negative bacteria. These periplasmic spaces are relatively thick and contain a thin peptidoglycan layer (PGL), also referred to as a thin cell wall.